enzyme binding [GO:0019899] (MF) Definition: Binding to an enzyme, a protein with catalytic activity. Sources: GOC:jl Relationships: is_a protein binding [GO:0005515] Subtypes: protease binding [GO:0002020], GO:0008179, thioglucosidase binding [GO:0010180], DEAD/H-box RNA helicase binding [GO:0017151], kinase binding [GO:0019900], phosphatase binding [GO:0019902], thioesterase binding [GO:0031996], succinate-semialdehyde dehydrogenase binding [GO:0032145], acrosin binding [GO:0032190], histone acetyltransferase binding [GO:0035035], glutamate-cysteine ligase catalytic subunit binding [GO:0035226], zymogen binding [GO:0035375], lipase binding [GO:0035473], histone deacetylase binding [GO:0042826], phospholipase binding [GO:0043274], small protein activating enzyme binding [GO:0044388], ubiquitin-like protein ligase binding [GO:0044389], ubiquitin-like protein conjugating enzyme binding [GO:0044390], DNA topoisomerase binding [GO:0044547], GTP cyclohydrolase binding [GO:0044549], nitric-oxide synthase binding [GO:0050998], GTPase binding [GO:0051020], ATPase binding [GO:0051117], RNA polymerase binding [GO:0070063], DNA polymerase binding [GO:0070182], peptidyl-proline 4-dioxygenase binding [GO:0098650], GO:1990226, GO:1990827